negative regulation of serotonin secretion [GO:0014063] (biological process) Definition: Any process that stops, prevents, or reduces the frequency, rate or extent of the regulated release of serotonin. Also known as: down regulation of serotonin secretion, down-regulation of serotonin secretion, downregulation of serotonin secretion, inhibition of serotonin secretion, positive regulation of serotonin release Sources: GOC:ef Relationships: is a type of regulation of serotonin secretion [GO:0014062]; is a type of negative regulation of monoatomic ion transport [GO:0043271]; is_a negative regulation of secretion by cell [GO:1903531]; negatively regulates GO:0001820